SUMO binding [GO:0032183] (molecular function) Subtypes: SUMO polymer binding [GO:0032184] Sources: GOC:mah Also known as: Smt3 monomer binding, Smt3 binding Definition: Binding to the small ubiquitin-like protein SUMO. Relationships: is a type of ubiquitin-like protein binding [GO:0032182]